{
  "term_id": "GO:0061630",
  "gene_name": "E3 ubiquitin-protein ligase TRIM71",
  "term_label": "ubiquitin protein ligase activity",
  "gene": "UniProtKB:Q2Q1W2",
  "gene_symbol": "TRIM71"
}